regulation of keratinocyte differentiation [GO:0045616] (biological process) Subtypes: GO:0045617, positive regulation of keratinocyte differentiation [GO:0045618] Relationships: is a type of regulation of epidermal cell differentiation [GO:0045604]; regulates keratinocyte differentiation [GO:0030216] Definition: Any process that modulates the frequency, rate or extent of keratinocyte differentiation. Sources: GOC:go_curators